{
  "term_id": "GO:0000122",
  "gene_name": "Chromobox protein homolog 2",
  "gene_symbol": "CBX2",
  "gene": "UniProtKB:Q14781",
  "term_label": "negative regulation of transcription by RNA polymerase II"
}